{
  "term_id": "GO:0006954",
  "term_label": "inflammatory response",
  "gene_name": "C-C motif chemokine 24",
  "gene_symbol": "CCL24",
  "gene": "UniProtKB:O00175"
}